{
  "gene_name": "WD repeat-containing protein 7",
  "term_label": "cytoplasm",
  "term_id": "GO:0005737",
  "gene_symbol": "WDR7",
  "gene": "UniProtKB:Q9Y4E6"
}